{
  "gene_symbol": "FADD",
  "term_id": "GO:0097191",
  "term_label": "extrinsic apoptotic signaling pathway",
  "gene": "UniProtKB:Q13158",
  "gene_name": "FAS-associated death domain protein"
}